negative regulation of interleukin-9 production [GO:0032718] (biological process) Relationships: is a type of negative regulation of cytokine production [GO:0001818]; is a type of regulation of interleukin-9 production [GO:0032678]; negatively regulates interleukin-9 production [GO:0032638] Sources: GOC:mah Also known as: down regulation of interleukin-9 production, down-regulation of interleukin-9 production, downregulation of interleukin-9 production, negative regulation of IL-9 production, inhibition of interleukin-9 production, negative regulation of interleukin-9 biosynthetic process Definition: Any process that stops, prevents, or reduces the frequency, rate, or extent of interleukin-9 production.